pericardium morphogenesis [GO:0003344] (biological process) Relationships: is a type of morphogenesis of an epithelial sheet [GO:0002011]; is a type of embryonic morphogenesis [GO:0048598]; is part of pericardium development [GO:0060039] References: PMID:18722343 Sources: GOC:dph Definition: The process in which the anatomical structure of the pericardium is generated and organized.